{
  "gene": "UniProtKB:Q5T2W1",
  "term_label": "protein localization to plasma membrane",
  "gene_symbol": "PDZK1",
  "term_id": "GO:0072659",
  "gene_name": "Na(+)_H(+) exchange regulatory cofactor NHE-RF3"
}